carotenoid metabolic process [GO:0016116] (biological process) Sources: ISBN:0198547684 Relationships: is a type of terpenoid metabolic process [GO:0006721] Subtypes: GO:0016117, carotenoid catabolic process [GO:0016118], GO:0016122, beta-carotene metabolic process [GO:1901810] Definition: The chemical reactions and pathways involving carotenoids, tetraterpenoid compounds in which two units of 4 isoprenoid residues joined head-to-tail are themselves joined tail-to-tail. Also known as: carotenoid metabolism